nicotinic acid riboside hydrolase activity [GO:0070636] (molecular function) Definition: Catalysis of the reaction: nicotinic acid riboside + H2O = nicotinic acid + D-ribose. Also known as: D-ribosylnicotinate hydrolase activity, D-ribosylnicotinic acid hydrolase activity, nicotinate ribonucleoside hydrolase activity, nicotinate riboside hydrolase activity, nicotinic acid ribonucleoside hydrolase activity Relationships: is_a hydrolase activity, hydrolyzing N-glycosyl compounds [GO:0016799] References: PMID:19001417 Sources: GOC:mah